{
  "term_label": "double-stranded DNA 3'-5' DNA exonuclease activity",
  "gene_symbol": "APEX2",
  "gene": "UniProtKB:Q9UBZ4",
  "gene_name": "DNA-(apurinic or apyrimidinic site) endonuclease 2",
  "term_id": "GO:0008311"
}